{
  "term_id": "GO:0044208",
  "gene_name": "Adenylosuccinate synthetase isozyme 1",
  "gene_symbol": "ADSS1",
  "gene": "UniProtKB:Q8N142",
  "term_label": "'de novo' AMP biosynthetic process"
}